visual perception involved in equilibrioception [GO:0051356] (biological process) Also known as: perception of orientation with respect to gravity by visual perception, equilibrioception by visual perception, visual perception during equilibrioception Relationships: is a type of GO:0007601; is part of equilibrioception [GO:0050957] Sources: GOC:ai Definition: The series of events during equilibrioception required for an organism to receive a visual stimulus, convert it to a molecular signal, and recognize and characterize the signal. Visual input plays an important role in the ability of an organism to perceive its orientation with respect to gravity.